prostaglandin secretion [GO:0032310] (biological process) Subtypes: prostaglandin secretion involved in immune response [GO:0090323], GO:0100009 Definition: The regulated release of a prostaglandin, any of a group of biologically active metabolites which contain a cyclopentane ring, from a cell or a tissue. Regulation: regulated by regulation of prostaglandin secretion [GO:0032306]; negatively regulated by GO:0032307; positively regulated by positive regulation of prostaglandin secretion [GO:0032308] Relationships: is a type of prostaglandin transport [GO:0015732]; is a type of GO:0023061; is a type of icosanoid secretion [GO:0032309]; is a type of lipid export from cell [GO:0140353] Sources: GOC:mah Also known as: prostacyclin secretion